{
  "gene": "UniProtKB:Q9UKT6",
  "gene_name": "Putative F-box_LRR-repeat protein 21",
  "term_id": "GO:0005829",
  "term_label": "cytosol",
  "gene_symbol": "FBXL21P"
}